{
  "gene": "UniProtKB:Q96G61",
  "gene_name": "Diphosphoinositol polyphosphate phosphohydrolase 3-beta",
  "term_label": "bis(5'-adenosyl)-hexaphosphatase activity",
  "term_id": "GO:0034431",
  "gene_symbol": "NUDT11"
}